{
  "term_label": "nucleus",
  "gene_symbol": "EIF1AD",
  "term_id": "GO:0005634",
  "gene_name": "Probable RNA-binding protein EIF1AD",
  "gene": "UniProtKB:Q8N9N8"
}